{
  "gene_symbol": "FNIP2",
  "term_id": "UNKNOWN:0002",
  "gene": "UniProtKB:Q9P278",
  "term_label": "Unknown biological process",
  "gene_name": "Folliculin-interacting protein 2"
}